zonula adherens assembly [GO:0045186] (biological process) Definition: Assembly of the zonula adherens, a cell-cell adherens junction which forms a continuous belt near the apex of epithelial cells. Relationships: is a type of adherens junction assembly [GO:0034333]; is part of apical junction assembly [GO:0043297] Sources: GOC:bf